embryonic heart tube dorsal/ventral pattern formation [GO:0060970] (biological process) Sources: GOC:mtg_heart Definition: The regionalization process in which the areas along the dorsal/ventral axis of the embryonic heart tube are established. This process will determine the patterns of cell differentiation along the axis. Relationships: is a type of dorsal/ventral pattern formation [GO:0009953]; is part of embryonic heart tube development [GO:0035050]